{
  "term_label": "cell differentiation",
  "term_id": "GO:0030154",
  "gene": "UniProtKB:Q06546",
  "gene_name": "GA-binding protein alpha chain",
  "gene_symbol": "GABPA"
}